{
  "gene": "UniProtKB:P35237",
  "term_label": "serine-type endopeptidase inhibitor activity",
  "gene_name": "Serpin B6",
  "term_id": "GO:0004867",
  "gene_symbol": "SERPINB6"
}